{
  "gene": "UniProtKB:P61129",
  "term_id": "GO:0005654",
  "gene_symbol": "ZC3H6",
  "term_label": "nucleoplasm",
  "gene_name": "Zinc finger CCCH domain-containing protein 6"
}